{
  "gene": "UniProtKB:O75170",
  "gene_symbol": "PPP6R2",
  "gene_name": "Serine_threonine-protein phosphatase 6 regulatory subunit 2",
  "term_label": "regulation of signal transduction",
  "term_id": "GO:0009966"
}